{
  "gene_symbol": "H1-10",
  "gene_name": "Histone H1.10",
  "term_label": "chromosome condensation",
  "term_id": "GO:0030261",
  "gene": "UniProtKB:Q92522"
}